alkene biosynthetic process [GO:0043450] (biological process) Relationships: is a type of GO:1900674 Also known as: alkene anabolism, alkene biosynthesis, alkene formation, alkene synthesis Sources: GOC:jl, Wikipedia:Alkene Subtypes: GO:0009693, GO:1900682, GO:1900873, GO:1900875, nonadec-1-ene biosynthetic process [GO:1900877], GO:1900881, GO:1900883, 1-undecene biosynthetic process [GO:1902821] Definition: The chemical reactions and pathways resulting in the formation of an alkene, any acyclic branched or unbranched hydrocarbon having one carbon-carbon double bond and the general formula CnH2n.